{
  "term_label": "heart development",
  "gene_name": "Protein HEG homolog 1",
  "gene_symbol": "HEG1",
  "gene": "UniProtKB:Q9ULI3",
  "term_id": "GO:0007507"
}